{
  "gene": "UniProtKB:P20340",
  "term_label": "Golgi apparatus",
  "gene_symbol": "RAB6A",
  "term_id": "GO:0005794",
  "gene_name": "Ras-related protein Rab-6A"
}